oxidoreductase activity, acting on metal ions, NAD or NADP as acceptor [GO:0016723] (MF) Also known as: oxidoreductase activity, oxidizing metal ions, NAD or NADP as acceptor, oxidoreductase activity, reducing metal ions, NAD or NADP as acceptor Definition: Catalysis of an oxidation-reduction in which the metal ion is reduced and NAD+ or NADP+ acts as an electron acceptor. Relationships: is a type of oxidoreductase activity, acting on metal ions [GO:0016722] Subtypes: cupric reductase (NADH) activity [GO:0008823], GO:0016152, [methionine synthase] reductase (NADPH) activity [GO:0030586], cyanocobalamin reductase (cyanide-eliminating) (NADP+) activity [GO:0033787], GO:0047852, ferric-chelate reductase (NADPH) activity [GO:0052851], GO:0140618 Sources: GOC:mah